{
  "gene": "UniProtKB:Q9Y5F9",
  "term_label": "cell adhesion",
  "term_id": "GO:0007155",
  "gene_symbol": "PCDHGB6",
  "gene_name": "Protocadherin gamma-B6"
}